{
  "term_label": "metalloendopeptidase activity",
  "gene": "UniProtKB:P52888",
  "term_id": "GO:0004222",
  "gene_symbol": "THOP1",
  "gene_name": "Thimet oligopeptidase"
}